{
  "gene_symbol": "CCDC42",
  "term_id": "UNKNOWN:0001",
  "gene": "UniProtKB:Q96M95",
  "gene_name": "Coiled-coil domain-containing protein 42",
  "term_label": "Unknown molecular function"
}